5'-(N(7)-methyl 5'-triphosphoguanosine)-[mRNA] diphosphatase activity [GO:0140932] (molecular function) References: PMID:24742626, PMID:32723815 Also known as: m(7)GpppN m(7)GMP phosphohydrolase activity, m(7)GpppX diphosphatase activity, m(7)GpppX pyrophosphatase activity Definition: Catalysis of the reaction: a 5'-end (N2,N2,N7-trimethyl 5'-triphosphoguanosine)-ribonucleoside in mRNA + H2O = a 5'-end diphospho-ribonucleoside in mRNA + 2 H+ + N7-methyl-GMP. Can also use (N7-methyl 5'-triphosphoguanosine)-ribonucleoside in mRNA as a substrate. Relationships: is a type of pyrophosphatase activity [GO:0016462]